{
  "gene": "UniProtKB:Q69YN4",
  "gene_symbol": "VIRMA",
  "term_label": "Unknown biological process",
  "gene_name": "Protein virilizer homolog",
  "term_id": "UNKNOWN:0002"
}